3-hydroxyanthranilate 3,4-dioxygenase activity [GO:0000334] (molecular function) Relationships: is a type of oxidoreductase activity, acting on single donors with incorporation of molecular oxygen, incorporation of two atoms of oxygen [GO:0016702] Also known as: 3-hydroxyanthranilate oxygenase activity, 3-hydroxyanthranilate:oxygen 3,4-oxidoreductase (decyclizing), 3-hydroxyanthranilic acid dioxygenase activity, 3-hydroxyanthranilic acid oxygenase activity, 3-hydroxyanthranilic oxygenase activity, 3HAO Sources: EC:1.13.11.6, RHEA:17953 Definition: Catalysis of the reaction: 3-hydroxyanthranilate + O2 = cis,cis-2-amino-3-(3-oxoprop-1-enyl)but-2-enedioate + H+.